{
  "gene_symbol": "SYTL5",
  "term_label": "exocytic vesicle",
  "gene": "UniProtKB:Q8TDW5",
  "gene_name": "Synaptotagmin-like protein 5",
  "term_id": "GO:0070382"
}